{
  "gene_symbol": "AIF1L",
  "term_id": "GO:0005509",
  "gene": "UniProtKB:Q9BQI0",
  "gene_name": "Allograft inflammatory factor 1-like",
  "term_label": "calcium ion binding"
}